{
  "term_label": "guanyl-nucleotide exchange factor activity",
  "gene_symbol": "DENND5B",
  "gene_name": "DENN domain-containing protein 5B",
  "gene": "UniProtKB:Q6ZUT9",
  "term_id": "GO:0005085"
}